symbiont-mediated perturbation of host cell-cell junction [GO:0044067] (biological process) Also known as: disruption of host cell-cell junction, modification by symbiont of host cell-cell junction, modification by symbiont of host intercellular junctions, modification of host intercellular junctions by symbiont, modification of host cell-cell junction, symbiont-mediated disruption of host cell-cell junction Relationships: is a type of symbiont-mediated disruption of host cellular anatomical structure [GO:0052008] Definition: The process in which an organism effects a change that impairs the structure or temporarily subverts the host intercellular junction. Intercellular junction include tight junctions and adherens junctions. References: PMID:16102958 Subtypes: GO:0098865